{
  "gene_symbol": "PGM3",
  "term_id": "GO:0004610",
  "gene_name": "Phosphoacetylglucosamine mutase",
  "gene": "UniProtKB:O95394",
  "term_label": "phosphoacetylglucosamine mutase activity"
}